{
  "term_label": "endosome",
  "term_id": "GO:0005768",
  "gene_symbol": "PACSIN3",
  "gene": "UniProtKB:Q9UKS6",
  "gene_name": "Protein kinase C and casein kinase substrate in neurons protein 3"
}